{
  "term_label": "Unknown molecular function",
  "term_id": "UNKNOWN:0001",
  "gene_symbol": "SYCP3",
  "gene": "UniProtKB:Q8IZU3",
  "gene_name": "Synaptonemal complex protein 3"
}